{
  "term_id": "GO:0051464",
  "gene_symbol": "CRH",
  "term_label": "positive regulation of cortisol secretion",
  "gene_name": "Corticoliberin",
  "gene": "UniProtKB:P06850"
}